{
  "gene": "UniProtKB:O96009",
  "term_label": "lysosome",
  "gene_symbol": "NAPSA",
  "gene_name": "Napsin-A",
  "term_id": "GO:0005764"
}